{
  "term_id": "GO:0004843",
  "gene_symbol": "USP34",
  "gene_name": "Ubiquitin carboxyl-terminal hydrolase 34",
  "term_label": "cysteine-type deubiquitinase activity",
  "gene": "UniProtKB:Q70CQ2"
}